DNA methyltransferase complex [GO:0140020] (cellular component) Definition: A protein complex that possesses DNA methyltransferase activity. References: PMID:20939822, PMID:24947342 Relationships: is a type of methyltransferase complex [GO:0034708]